{
  "term_id": "GO:0120170",
  "gene": "UniProtKB:A0AVF1",
  "gene_name": "Intraflagellar transport protein 56",
  "gene_symbol": "IFT56",
  "term_label": "intraciliary transport particle B binding"
}